aspartate 4-decarboxylase activity [GO:0047688] (molecular function) Definition: Catalysis of the reaction: L-aspartate = L-alanine + CO2. Sources: EC:4.1.1.12, MetaCyc:ASPARTATE-4-DECARBOXYLASE-RXN Also known as: L-aspartate 4-carboxy-lyase (L-alanine-forming), L-aspartate 4-carboxy-lyase activity, L-aspartate beta-decarboxylase activity, L-cysteine sulfinate acid desulfinase activity, aminomalonic decarboxylase activity, aspartate beta-decarboxylase activity, aspartate omega-decarboxylase activity, aspartic beta-decarboxylase activity, aspartic omega-decarboxylase activity, cysteine sulfinic desulfinase activity, desulfinase activity Relationships: is a type of GO:0016831